{
  "term_id": "UNKNOWN:0001",
  "term_label": "Unknown molecular function",
  "gene_name": "Zinc fingers and homeoboxes protein 1, isoform 2",
  "gene_symbol": "ZHX1-C8orf76",
  "gene": "UniProtKB:Q96EF9"
}